{
  "gene": "UniProtKB:O95210",
  "term_label": "Unknown biological process",
  "gene_name": "Starch-binding domain-containing protein 1",
  "term_id": "UNKNOWN:0002",
  "gene_symbol": "STBD1"
}